{
  "term_id": "GO:0004930",
  "gene_symbol": "FFAR2",
  "term_label": "G protein-coupled receptor activity",
  "gene_name": "Free fatty acid receptor 2",
  "gene": "UniProtKB:O15552"
}